{
  "term_id": "GO:0050821",
  "term_label": "protein stabilization",
  "gene_symbol": "OTUD3",
  "gene": "UniProtKB:Q5T2D3",
  "gene_name": "OTU domain-containing protein 3"
}